{
  "gene": "UniProtKB:O75928",
  "term_label": "regulation of transcription by RNA polymerase II",
  "gene_name": "E3 SUMO-protein ligase PIAS2",
  "term_id": "GO:0006357",
  "gene_symbol": "PIAS2"
}